{
  "gene_name": "ATP synthase-coupling factor 6, mitochondrial",
  "gene_symbol": "ATP5PF",
  "term_label": "Unknown biological process",
  "term_id": "UNKNOWN:0002",
  "gene": "UniProtKB:P18859"
}